{
  "gene_name": "Abl interactor 2",
  "gene_symbol": "ABI2",
  "term_id": "GO:0048858",
  "gene": "UniProtKB:Q9NYB9",
  "term_label": "cell projection morphogenesis"
}